{
  "gene": "UniProtKB:P33121",
  "gene_symbol": "ACSL1",
  "term_id": "GO:0035338",
  "term_label": "long-chain fatty-acyl-CoA biosynthetic process",
  "gene_name": "Long-chain-fatty-acid--CoA ligase 1"
}